{
  "term_label": "osteoclast differentiation",
  "gene_name": "Ephrin-A2",
  "gene_symbol": "EFNA2",
  "gene": "UniProtKB:O43921",
  "term_id": "GO:0030316"
}